{
  "gene": "UniProtKB:Q08AE8",
  "gene_name": "Protein spire homolog 1",
  "term_label": "establishment of meiotic spindle localization",
  "gene_symbol": "SPIRE1",
  "term_id": "GO:0051295"
}